{
  "term_label": "sterol metabolic process",
  "gene": "UniProtKB:Q9HAW9",
  "gene_name": "UDP-glucuronosyltransferase 1A8",
  "term_id": "GO:0016125",
  "gene_symbol": "UGT1A8"
}